{
  "gene_symbol": "MTUS2",
  "term_label": "microtubule binding",
  "gene_name": "Microtubule-associated tumor suppressor candidate 2",
  "term_id": "GO:0008017",
  "gene": "UniProtKB:Q5JR59"
}